alpha9-beta1 integrin-ADAM15 complex [GO:0071056] (cellular component) Relationships: is a type of plasma membrane protein complex [GO:0098797] References: PMID:11882657 Definition: A protein complex that consists of an alpha9-beta1 integrin complex bound to the transmembrane metallopeptidase ADAM15. Also known as: ITGA9-ITGB1-ADAM15 complex